selenate reductase activity [GO:0033797] (molecular function) Definition: Catalysis of the reaction: 2 e(-) + 2 H+ + selenate = H2O + selenite. Also known as: selenite:reduced acceptor oxidoreductase activity Sources: RHEA:14029 Relationships: is a type of oxidoreductase activity [GO:0016491]